{
  "term_id": "GO:1904263",
  "term_label": "positive regulation of TORC1 signaling",
  "gene": "UniProtKB:O60478",
  "gene_symbol": "GPR137B",
  "gene_name": "Integral membrane protein GPR137B"
}